{
  "gene": "UniProtKB:Q2M3M2",
  "term_label": "transmembrane transporter activity",
  "gene_name": "Sodium_glucose cotransporter 4",
  "term_id": "GO:0022857",
  "gene_symbol": "SLC5A9"
}